{
  "gene": "UniProtKB:Q9BSF8",
  "term_id": "UNKNOWN:0001",
  "term_label": "Unknown molecular function",
  "gene_symbol": "BTBD10",
  "gene_name": "BTB_POZ domain-containing protein 10"
}